{
  "term_label": "basement membrane",
  "gene": "UniProtKB:A4D0S4",
  "gene_name": "Laminin subunit beta-4",
  "term_id": "GO:0005604",
  "gene_symbol": "LAMB4"
}